{
  "gene": "UniProtKB:Q86UK0",
  "term_label": "Unknown cellular component",
  "gene_symbol": "ABCA12",
  "term_id": "UNKNOWN:0003",
  "gene_name": "Glucosylceramide transporter ABCA12"
}